rRNA (cytosine) methyltransferase activity [GO:0016434] (MF) Definition: Catalysis of the reaction: S-adenosyl-L-methionine + rRNA = S-adenosyl-L-homocysteine + rRNA containing methylcytosine. Sources: GOC:go-curators Relationships: is a type of rRNA methyltransferase activity [GO:0008649] Subtypes: rRNA (cytosine-C5-)-methyltransferase activity [GO:0009383], rRNA (cytosine-2'-O-)-methyltransferase activity [GO:0070677], rRNA (cytosine-N4-)-methyltransferase activity [GO:0071424]